{
  "term_id": "GO:0007169",
  "gene_name": "Tyrosine-protein kinase Fyn",
  "gene_symbol": "FYN",
  "gene": "UniProtKB:P06241",
  "term_label": "cell surface receptor protein tyrosine kinase signaling pathway"
}